{
  "term_label": "Unknown cellular component",
  "term_id": "UNKNOWN:0003",
  "gene_symbol": "FAM166A",
  "gene": "UniProtKB:Q6J272",
  "gene_name": "Protein FAM166A"
}